host-mediated activation of viral genome replication [GO:0044829] (biological process) Sources: GOC:jl Relationships: is a type of host-mediated activation of viral process [GO:0044794]; is_a GO:0044827 Also known as: positive regulation by host of viral genome replication Definition: A process in which a host organism initiates, promotes, or enhances the normal execution of viral genome replication.